{
  "term_label": "Unknown molecular function",
  "gene": "UniProtKB:P0CL83",
  "term_id": "UNKNOWN:0001",
  "gene_name": "Putative STAG3-like protein 1",
  "gene_symbol": "STAG3L1"
}